{
  "gene_symbol": "LY96",
  "term_label": "lipopolysaccharide immune receptor activity",
  "term_id": "GO:0001875",
  "gene": "UniProtKB:Q9Y6Y9",
  "gene_name": "Lymphocyte antigen 96"
}